{
  "gene_symbol": "MYNN",
  "term_id": "GO:0000978",
  "gene": "UniProtKB:Q9NPC7",
  "term_label": "RNA polymerase II cis-regulatory region sequence-specific DNA binding",
  "gene_name": "Myoneurin"
}